cell-substrate junction organization [GO:0150115] (biological process) Relationships: is_a GO:0034330 Regulation: regulated by GO:0150116; positively regulated by GO:0150117; negatively regulated by GO:0150118 Definition: A process that is carried out at the cellular level which results in the assembly, arrangement of constituent parts, or disassembly of a cell-substrate junction. A cell-substrate junction is a specialized region of connection between a cell and the extracellular matrix. Subtypes: GO:0007044, cell-substrate junction disassembly [GO:0120180] References: PMID:10419689, PMID:1643657, PMID:16805308, PMID:26923917, PMID:8314002 Sources: GOC:aruk, GOC:bc